{
  "gene_symbol": "SLC13A1",
  "term_id": "GO:0006814",
  "gene_name": "Solute carrier family 13 member 1",
  "term_label": "sodium ion transport",
  "gene": "UniProtKB:Q9BZW2"
}